high-density lipoprotein particle receptor activity [GO:0070506] (molecular function) Relationships: is a type of lipoprotein particle receptor activity [GO:0030228]; has part high-density lipoprotein particle binding [GO:0008035] References: PMID:9211901 Sources: GOC:BHF, GOC:bf, GOC:rl Also known as: HDL receptor, high-density lipoprotein receptor activity Definition: Combining with a high-density lipoprotein particle and delivering the high-density lipoprotein into the cell via endocytosis.